{
  "term_id": "GO:0005759",
  "gene": "UniProtKB:O75127",
  "term_label": "mitochondrial matrix",
  "gene_name": "Pentatricopeptide repeat-containing protein 1, mitochondrial",
  "gene_symbol": "PTCD1"
}